{
  "gene_name": "Serine_threonine-protein kinase haspin",
  "gene": "UniProtKB:Q8TF76",
  "term_label": "nucleus",
  "term_id": "GO:0005634",
  "gene_symbol": "HASPIN"
}